induction of synaptic plasticity by chemical substance [GO:0051915] (biological process) Also known as: activation of synaptic plasticity by chemical substance, activation of synaptic plasticity by drug, induction of synaptic plasticity by drug Sources: GOC:ai Definition: The process in which a chemical substance activates synaptic plasticity, the ability of synapses to change as circumstances require. Relationships: is_a positive regulation of synaptic plasticity by chemical substance [GO:0051914]